beta-lactamase activity [GO:0008800] (molecular function) Definition: Catalysis of the reaction: a beta-lactam + H2O = a substituted beta-amino acid. Also known as: ampicillinase activity, beta-lactam hydrolase activity, beta-lactamase A, B, C, beta-lactamase AME I, beta-lactamase I-III, cephalosporin-beta-lactamase activity, exopenicillinase activity, neutrapen, penicillin amido-beta-lactamhydrolase activity, penicillin beta-lactamase activity, penicillinase I, II Regulation: regulated by regulation of beta-lactamase activity [GO:0033252] Sources: EC:3.5.2.6 Relationships: is a type of hydrolase activity, acting on carbon-nitrogen (but not peptide) bonds, in cyclic amides [GO:0016812]